{
  "term_id": "UNKNOWN:0003",
  "gene": "UniProtKB:Q2M2E3",
  "term_label": "Unknown cellular component",
  "gene_name": "Outer dense fiber protein 4",
  "gene_symbol": "ODF4"
}